{
  "gene_name": "Tubulin alpha 3f pseudogene",
  "term_id": "UNKNOWN:0003",
  "gene_symbol": "TUBA3FP",
  "term_label": "Unknown cellular component",
  "gene": "UniProtKB:A0A994J5G1"
}